{
  "gene_name": "Calcium homeostasis endoplasmic reticulum protein",
  "term_id": "GO:0048471",
  "term_label": "perinuclear region of cytoplasm",
  "gene": "UniProtKB:Q8IWX8",
  "gene_symbol": "CHERP"
}